{
  "term_label": "cytosol",
  "term_id": "GO:0005829",
  "gene": "UniProtKB:Q13162",
  "gene_symbol": "PRDX4",
  "gene_name": "Peroxiredoxin-4"
}